{
  "gene_name": "Protein Wnt-5a",
  "gene": "UniProtKB:P41221",
  "term_id": "GO:0045165",
  "gene_symbol": "WNT5A",
  "term_label": "cell fate commitment"
}